{
  "gene_symbol": "UGT2B15",
  "gene_name": "UDP-glucuronosyltransferase 2B15",
  "term_id": "GO:0008210",
  "term_label": "estrogen metabolic process",
  "gene": "UniProtKB:P54855"
}